{
  "term_id": "UNKNOWN:0002",
  "gene_name": "Large ribosomal subunit protein uL4",
  "term_label": "Unknown biological process",
  "gene": "UniProtKB:P36578",
  "gene_symbol": "RPL4"
}